response to anticoagulant [GO:0061476] (BP) Definition: Any process that results in a change in state or activity of a cell or an organism (in terms of movement, secretion, enzyme production, gene expression, etc.) as a result of an anticoagulant stimulus. Sources: GOC:dph Relationships: is a type of response to chemical [GO:0042221]